thiocyanate catabolic process [GO:0046265] (biological process) Definition: The chemical reactions and pathways resulting in the breakdown of thiocyanate, any anion of thiocyanic acid. Sources: GOC:ai Also known as: thiocyanate breakdown, thiocyanate catabolism, thiocyanate degradation Relationships: is a type of thiocyanate metabolic process [GO:0018969]; is a type of xenobiotic catabolic process [GO:0042178]; is a type of GO:0044273; is a type of GO:0044282